mesonephric glomerular parietal epithelial cell development [GO:0061254] (biological process) Sources: GOC:mtg_kidney_jan10 Relationships: is a type of GO:0061251; is a type of glomerular parietal epithelial cell development [GO:0072016]; is part of mesonephric glomerular parietal epithelial cell differentiation [GO:0061253] Definition: The process whose specific outcome is the progression of a mesonephric glomerular parietal epithelial cell over time, from its formation to the mature structure. Mesonephric glomerular parietal epithelial cells are specialized epithelial cells that form tight junctions as a barrier to protein transport.